platelet dense granule organization [GO:0060155] (biological process) Relationships: is a type of secretory granule organization [GO:0033363] Also known as: platelet dense granule organisation, bull's eye body organization and biogenesis, platelet dense body organization and biogenesis, platelet dense granule organization and biogenesis References: PMID:11487378 Sources: GOC:dph Definition: A process that is carried out at the cellular level which results in the assembly, arrangement of constituent parts, or disassembly of a platelet dense granule. A platelet dense granule is an electron-dense granule occurring in blood platelets that stores and secretes adenosine nucleotides and serotonin. They contain a highly condensed core consisting of serotonin, histamine, calcium, magnesium, ATP, ADP, pyrophosphate and membrane lysosomal proteins.